{
  "gene": "UniProtKB:P40199",
  "term_id": "UNKNOWN:0001",
  "gene_name": "Carcinoembryonic antigen-related cell adhesion molecule 6",
  "term_label": "Unknown molecular function",
  "gene_symbol": "CEACAM6"
}